androgen metabolic process [GO:0008209] (biological process) Sources: ISBN:0198506732 Relationships: is_a GO:0008202; is_a GO:0042445 Also known as: androgen metabolism Definition: The chemical reactions and pathways involving androgens, C19 steroid hormones that can stimulate the development of male sexual characteristics. Subtypes: androgen biosynthetic process [GO:0006702], androgen catabolic process [GO:0006710]